{
  "gene_name": "Putative glutathione hydrolase light chain 3",
  "gene_symbol": "GGTLC3",
  "gene": "UniProtKB:B5MD39",
  "term_id": "UNKNOWN:0003",
  "term_label": "Unknown cellular component"
}